compound eye cone cell fate specification [GO:0042679] (biological process) Regulation: regulated by regulation of compound eye cone cell fate specification [GO:0042682]; negatively regulated by GO:0042683 Sources: GOC:mtg_sensu Definition: The process in which a cell becomes capable of differentiating autonomously into a compound eye cone cell in an environment that is neutral with respect to the developmental pathway; upon specification, the cell fate can be reversed. Relationships: is a type of cell fate specification [GO:0001708]; is part of compound eye cone cell fate commitment [GO:0042676]